{
  "term_id": "GO:0005634",
  "gene_symbol": "KCNIP3",
  "gene_name": "Calsenilin",
  "gene": "UniProtKB:Q9Y2W7",
  "term_label": "nucleus"
}